{
  "gene": "UniProtKB:Q8NGD1",
  "term_label": "Unknown biological process",
  "gene_symbol": "OR4N2",
  "term_id": "UNKNOWN:0002",
  "gene_name": "Olfactory receptor 4N2"
}